{
  "gene_symbol": "DUSP29",
  "gene": "UniProtKB:Q68J44",
  "term_label": "MAP kinase phosphatase activity",
  "term_id": "GO:0033549",
  "gene_name": "Dual specificity phosphatase 29"
}